{
  "gene": "UniProtKB:Q9ULR5",
  "term_id": "GO:0005737",
  "term_label": "cytoplasm",
  "gene_name": "Polyadenylate-binding protein-interacting protein 2B",
  "gene_symbol": "PAIP2B"
}